{
  "term_label": "Unknown cellular component",
  "gene_name": "Putative uncharacterized protein encoded by LINC00305",
  "term_id": "UNKNOWN:0003",
  "gene": "UniProtKB:Q7Z4B0",
  "gene_symbol": "LINC00305"
}